ribonucleoprotein granule [GO:0035770] (cellular component) References: PMID:16520386, PMID:20368989, PMID:21436445 Sources: GOC:go_curators, GOC:sp Subtypes: cytoplasmic ribonucleoprotein granule [GO:0036464], GO:0140168 Relationships: is a type of intracellular membraneless organelle [GO:0043232]; is a type of supramolecular complex [GO:0099080] Definition: A non-membranous macromolecular complex containing proteins and translationally silenced mRNAs. RNA granules contain proteins that control the localization, stability, and translation of their RNA cargo. Different types of RNA granules (RGs) exist, depending on the cell type and cellular conditions. Also known as: RNP granule, mRNP granule, RNA granule